negative regulation of B cell anergy [GO:0002671] (biological process) Subtypes: negative regulation of central B cell anergy [GO:0002915], negative regulation of peripheral B cell anergy [GO:0002918] Definition: Any process that stops, prevents, or reduces the frequency, rate, or extent of B cell anergy. Also known as: down regulation of B cell anergy, down-regulation of B cell anergy, downregulation of B cell anergy, negative regulation of B lymphocyte anergy, negative regulation of B-cell anergy, negative regulation of B-lymphocyte anergy, inhibition of B cell anergy Relationships: is a type of negative regulation of B cell tolerance induction [GO:0002662]; is a type of regulation of B cell anergy [GO:0002670]; is a type of negative regulation of lymphocyte anergy [GO:0002912]; negatively regulates GO:0002515 Sources: GOC:add